{
  "gene_name": "Vezatin",
  "gene_symbol": "VEZT",
  "gene": "UniProtKB:Q9HBM0",
  "term_id": "GO:0005886",
  "term_label": "plasma membrane"
}